{
  "gene_symbol": "GNAT3",
  "term_label": "sensory perception of sweet taste",
  "term_id": "GO:0050916",
  "gene_name": "Guanine nucleotide-binding protein G(t) subunit alpha-3",
  "gene": "UniProtKB:A8MTJ3"
}